{
  "gene_symbol": "HERPUD2",
  "gene_name": "Homocysteine-responsive endoplasmic reticulum-resident ubiquitin-like domain member 2 protein",
  "term_label": "Unknown cellular component",
  "gene": "UniProtKB:Q9BSE4",
  "term_id": "UNKNOWN:0003"
}